{
  "gene_symbol": "SEC14L3",
  "gene_name": "SEC14-like protein 3",
  "gene": "UniProtKB:Q9UDX4",
  "term_id": "GO:0005737",
  "term_label": "cytoplasm"
}